histone H3K9 deacetylase activity, hydrolytic mechanism [GO:0032129] (molecular function) Definition: Catalysis of the reaction: histone H3 N6-acetyl-L-lysine (position 9) + H2O = histone H3 L-lysine (position 9) + acetate. This reaction represents the removal of an acetyl group from lysine at position 9 of the histone H3 protein. References: PMID:28450737 Relationships: is a type of GO:0141050; is a type of histone deacetylase activity, hydrolytic mechanism [GO:0141221] Also known as: histone H3K9 deacetylase activity, histone H3-K9 deacetylase activity, histone deacetylase activity (H3-K9 specific)